{
  "term_id": "GO:0006357",
  "gene": "UniProtKB:O43296",
  "term_label": "regulation of transcription by RNA polymerase II",
  "gene_symbol": "ZNF264",
  "gene_name": "Zinc finger protein 264"
}